positive regulation of TRAIL-activated apoptotic signaling pathway [GO:1903984] (BP) Definition: Any process that activates or increases the frequency, rate or extent of TRAIL-activated apoptotic signaling pathway. References: PMID:24939851 Sources: GOC:PARL, GOC:TermGenie, GOC:bf, GO_REF:0000058 Also known as: positive regulation of TRAIL-activated extrinsic apoptotic signaling pathway, positive regulation of TRAIL-induced apoptotic signaling pathway, positive regulation of tumor necrosis factor-related apoptosis-inducing ligand apoptotic signaling pathway, up regulation of TRAIL-activated apoptotic signaling pathway, up regulation of TRAIL-activated extrinsic apoptotic signaling pathway, up regulation of TRAIL-induced apoptotic signaling pathway, up regulation of tumor necrosis factor-related apoptosis-inducing ligand apoptotic signaling pathway, up-regulation of TRAIL-activated apoptotic signaling pathway, up-regulation of TRAIL-activated extrinsic apoptotic signaling pathway, up-regulation of TRAIL-induced apoptotic signaling pathway, up-regulation of tumor necrosis factor-related apoptosis-inducing ligand apoptotic signaling pathway, upregulation of TRAIL-activated apoptotic signaling pathway, upregulation of TRAIL-activated extrinsic apoptotic signaling pathway, upregulation of TRAIL-induced apoptotic signaling pathway, upregulation of tumor necrosis factor-related apoptosis-inducing ligand apoptotic signaling pathway, activation of TRAIL-activated apoptotic signaling pathway, activation of TRAIL-activated extrinsic apoptotic signaling pathway, activation of TRAIL-induced apoptotic signaling pathway, activation of tumor necrosis factor-related apoptosis-inducing ligand apoptotic signaling pathway Relationships: is a type of positive regulation of extrinsic apoptotic signaling pathway via death domain receptors [GO:1902043]; is a type of GO:1903121; positively regulates TRAIL-activated apoptotic signaling pathway [GO:0036462]